{
  "term_label": "acyl-CoA metabolic process",
  "gene_symbol": "ACSM5",
  "term_id": "GO:0006637",
  "gene_name": "Acyl-coenzyme A synthetase ACSM5, mitochondrial",
  "gene": "UniProtKB:Q6NUN0"
}